{
  "gene_symbol": "VASN",
  "gene_name": "Vasorin",
  "gene": "UniProtKB:Q6EMK4",
  "term_label": "negative regulation of transforming growth factor beta receptor signaling pathway",
  "term_id": "GO:0030512"
}